{
  "gene_symbol": "CTPS1",
  "gene_name": "CTP synthase 1",
  "gene": "UniProtKB:P17812",
  "term_label": "pyrimidine nucleobase biosynthetic process",
  "term_id": "GO:0019856"
}